regulation of calcium ion transport into cytosol [GO:0010522] (biological process) Subtypes: negative regulation of calcium ion transport into cytosol [GO:0010523], positive regulation of calcium ion transport into cytosol [GO:0010524] Sources: GOC:dph, GOC:tb Relationships: is a type of regulation of cellular localization [GO:0060341]; is a type of regulation of biological quality [GO:0065008]; is a type of regulation of calcium ion transmembrane transport [GO:1903169]; regulates calcium ion transport into cytosol [GO:0060402] Definition: Any process that modulates the rate of the directed movement of calcium ions into the cytosol of a cell. The cytosol is that part of the cytoplasm that does not contain membranous or particulate subcellular components.